{
  "gene_symbol": "STARD3",
  "gene": "UniProtKB:Q14849",
  "gene_name": "StAR-related lipid transfer protein 3",
  "term_id": "GO:0140284",
  "term_label": "endoplasmic reticulum-endosome membrane contact site"
}